{
  "gene_name": "Zinc finger protein 879",
  "term_id": "GO:0000981",
  "gene_symbol": "ZNF879",
  "gene": "UniProtKB:B4DU55",
  "term_label": "DNA-binding transcription factor activity, RNA polymerase II-specific"
}